{
  "term_label": "box C/D sno(s)RNA 3'-end processing",
  "gene_symbol": "FBLL1",
  "gene": "UniProtKB:A6NHQ2",
  "term_id": "GO:0000494",
  "gene_name": "rRNA_tRNA 2'-O-methyltransferase fibrillarin-like protein 1"
}